{
  "term_label": "microtubule organizing center",
  "gene_name": "Centrosomal protein of 70 kDa",
  "gene_symbol": "CEP70",
  "gene": "UniProtKB:Q8NHQ1",
  "term_id": "GO:0005815"
}